{
  "gene": "UniProtKB:P27824",
  "term_label": "protein folding",
  "term_id": "GO:0006457",
  "gene_name": "Calnexin",
  "gene_symbol": "CANX"
}